{
  "gene_name": "Angiopoietin-related protein 7",
  "term_label": "Unknown molecular function",
  "term_id": "UNKNOWN:0001",
  "gene": "UniProtKB:O43827",
  "gene_symbol": "ANGPTL7"
}